{
  "gene": "UniProtKB:Q96B45",
  "term_label": "Unknown biological process",
  "term_id": "UNKNOWN:0002",
  "gene_symbol": "BORCS7",
  "gene_name": "BLOC-1-related complex subunit 7"
}